{
  "gene_symbol": "KRBA2",
  "gene": "UniProtKB:Q6ZNG9",
  "gene_name": "KRAB-A domain-containing protein 2",
  "term_label": "Unknown biological process",
  "term_id": "UNKNOWN:0002"
}